{
  "gene_name": "Sorting nexin-27",
  "term_label": "phosphatidylinositol binding",
  "gene": "UniProtKB:Q96L92",
  "term_id": "GO:0035091",
  "gene_symbol": "SNX27"
}